{
  "gene_name": "Bromodomain-containing protein 9",
  "term_label": "nucleus",
  "gene_symbol": "BRD9",
  "term_id": "GO:0005634",
  "gene": "UniProtKB:Q9H8M2"
}